{
  "gene_symbol": "TAS2R42",
  "term_label": "membrane",
  "term_id": "GO:0016020",
  "gene_name": "Taste receptor type 2 member 42",
  "gene": "UniProtKB:Q7RTR8"
}